positive regulation of hydrogen sulfide biosynthetic process [GO:1904828] (biological process) Also known as: positive regulation of hydrogen sulfide anabolism, positive regulation of hydrogen sulfide biosynthesis, positive regulation of hydrogen sulfide formation, positive regulation of hydrogen sulfide synthesis, positive regulation of hydrogen sulphide biosynthesis, positive regulation of hydrogen sulphide biosynthetic process, up regulation of hydrogen sulfide anabolism, up regulation of hydrogen sulfide biosynthesis, up regulation of hydrogen sulfide biosynthetic process, up regulation of hydrogen sulfide formation, up regulation of hydrogen sulfide synthesis, up regulation of hydrogen sulphide biosynthesis, up regulation of hydrogen sulphide biosynthetic process, up-regulation of hydrogen sulfide anabolism, up-regulation of hydrogen sulfide biosynthesis, up-regulation of hydrogen sulfide biosynthetic process, up-regulation of hydrogen sulfide formation, up-regulation of hydrogen sulfide synthesis, up-regulation of hydrogen sulphide biosynthesis, up-regulation of hydrogen sulphide biosynthetic process, upregulation of hydrogen sulfide anabolism, upregulation of hydrogen sulfide biosynthesis, upregulation of hydrogen sulfide biosynthetic process, upregulation of hydrogen sulfide formation, upregulation of hydrogen sulfide synthesis, upregulation of hydrogen sulphide biosynthesis, upregulation of hydrogen sulphide biosynthetic process, activation of hydrogen sulfide anabolism, activation of hydrogen sulfide biosynthesis, activation of hydrogen sulfide biosynthetic process, activation of hydrogen sulfide formation, activation of hydrogen sulfide synthesis, activation of hydrogen sulphide biosynthesis, activation of hydrogen sulphide biosynthetic process Relationships: is_a positive regulation of biosynthetic process [GO:0009891]; is a type of GO:1904826; positively regulates hydrogen sulfide biosynthetic process [GO:0070814] Definition: Any process that activates or increases the frequency, rate or extent of hydrogen sulfide biosynthetic process. References: PMID:22034194 Sources: GOC:BHF, GOC:BHF_miRNA, GOC:TermGenie, GOC:rph, GO_REF:0000058